alpha-glucoside transport [GO:0000017] (biological process) References: PMID:9919658 Sources: GOC:jl, ISBN:0198506732 Definition: The directed movement of alpha-glucosides into, out of or within a cell, or between cells, by means of some agent such as a transporter or pore. Alpha-glucosides are glycosides in which the sugar group is a glucose residue, and the anomeric carbon of the bond is in an alpha configuration. Relationships: is a type of glucoside transport [GO:0042946]